{
  "gene_name": "Runt-related transcription factor 1",
  "gene": "UniProtKB:Q01196",
  "gene_symbol": "RUNX1",
  "term_id": "GO:0030182",
  "term_label": "neuron differentiation"
}